{
  "gene_symbol": "HINT2",
  "gene": "UniProtKB:Q9BX68",
  "term_id": "UNKNOWN:0002",
  "gene_name": "Adenosine 5'-monophosphoramidase HINT2",
  "term_label": "Unknown biological process"
}